sensory system development [GO:0048880] (biological process) Sources: GOC:dgh Definition: The process whose specific outcome is the progression of a sensory system over time from its formation to the mature structure. Subtypes: lateral line system development [GO:0048925], GO:0150063, somatic sensory system development [GO:0160038] Relationships: is_a system development [GO:0048731]